{
  "gene_symbol": "SLCO2A1",
  "term_id": "GO:0015132",
  "gene_name": "Solute carrier organic anion transporter family member 2A1",
  "term_label": "prostaglandin transmembrane transporter activity",
  "gene": "UniProtKB:Q92959"
}